{
  "gene": "UniProtKB:Q9BYE2",
  "gene_symbol": "TMPRSS13",
  "term_label": "serine-type peptidase activity",
  "gene_name": "Transmembrane protease serine 13",
  "term_id": "GO:0008236"
}